{
  "term_label": "translational initiation",
  "gene_name": "Eukaryotic translation initiation factor 3 subunit D",
  "term_id": "GO:0006413",
  "gene_symbol": "EIF3D",
  "gene": "UniProtKB:O15371"
}